{
  "term_id": "GO:0001501",
  "term_label": "skeletal system development",
  "gene": "UniProtKB:Q96S86",
  "gene_symbol": "HAPLN3",
  "gene_name": "Hyaluronan and proteoglycan link protein 3"
}